{
  "term_label": "Unknown cellular component",
  "gene_symbol": "PLA2G2F",
  "term_id": "UNKNOWN:0003",
  "gene": "UniProtKB:Q9BZM2",
  "gene_name": "Group IIF secretory phospholipase A2"
}